mitochondrial ATP synthesis coupled electron transport [GO:0042775] (biological process) Definition: The transfer of electrons through a series of electron donors and acceptors, generating energy that is ultimately used for synthesis of ATP, as it occurs in the mitochondrial inner membrane or chloroplast thylakoid membrane. Relationships: is a type of GO:0042773; BFO_0000066 mitochondrion [GO:0005739] Regulation: regulated by regulation of mitochondrial ATP synthesis coupled electron transport [GO:1905446]; negatively regulated by negative regulation of mitochondrial ATP synthesis coupled electron transport [GO:1905447]; positively regulated by positive regulation of mitochondrial ATP synthesis coupled electron transport [GO:1905448] Sources: GOC:mtg_sensu, ISBN:0716731363 Also known as: mitochondrial electron transport, organelle ATP synthesis coupled electron transport